positive regulation of violaceol I biosynthetic process [GO:1900715] (biological process) Also known as: activation of violaceol I anabolism, activation of violaceol I biosynthesis, activation of violaceol I formation, activation of violaceol I synthesis, positive regulation of violaceol I anabolism, positive regulation of violaceol I biosynthesis, positive regulation of violaceol I formation, positive regulation of violaceol I synthesis, up regulation of violaceol I anabolism, up regulation of violaceol I biosynthesis, up regulation of violaceol I biosynthetic process, up regulation of violaceol I formation, up regulation of violaceol I synthesis, up-regulation of violaceol I anabolism, up-regulation of violaceol I biosynthesis, up-regulation of violaceol I biosynthetic process, up-regulation of violaceol I formation, up-regulation of violaceol I synthesis, upregulation of violaceol I anabolism, upregulation of violaceol I biosynthesis, upregulation of violaceol I biosynthetic process, upregulation of violaceol I formation, upregulation of violaceol I synthesis, activation of violaceol I biosynthetic process Sources: GOC:TermGenie, GOC:di Definition: Any process that activates or increases the frequency, rate or extent of violaceol I biosynthetic process. Relationships: is a type of GO:1900378; is a type of regulation of violaceol I biosynthetic process [GO:1900713]; positively regulates violaceol I biosynthetic process [GO:1900590]